{
  "gene": "UniProtKB:Q9H201",
  "gene_name": "Epsin-3",
  "gene_symbol": "EPN3",
  "term_id": "GO:0030125",
  "term_label": "clathrin vesicle coat"
}